{
  "term_id": "GO:0030154",
  "gene_symbol": "JAK1",
  "gene_name": "Tyrosine-protein kinase JAK1",
  "term_label": "cell differentiation",
  "gene": "UniProtKB:P23458"
}